venom-mediated reduction of heart rate [GO:0044556] (biological process) Relationships: is a type of venom-mediated perturbation of blood circulation [GO:0140134] Also known as: envenomation reducing heart rate, envenomation resulting in negative regulation of heart rate in another organism, envenomation resulting in negative regulation of heart rate of other organism, venom-mediated bradycardia, venom-mediated heart rate lowering Definition: A process in which an organism slows down the heart rate in another organism via the action of a venom. References: PMID:20923766, PMID:31370142 Sources: GOC:ecd, GOC:jl